{
  "gene_symbol": "MYT1",
  "gene": "UniProtKB:Q01538",
  "term_id": "UNKNOWN:0002",
  "gene_name": "Myelin transcription factor 1",
  "term_label": "Unknown biological process"
}